{
  "gene_name": "Zinc finger protein 836",
  "gene": "UniProtKB:Q6ZNA1",
  "term_label": "negative regulation of transcription by RNA polymerase II",
  "gene_symbol": "ZNF836",
  "term_id": "GO:0000122"
}